{
  "gene_name": "Zinc finger protein 148",
  "gene_symbol": "ZNF148",
  "term_id": "UNKNOWN:0003",
  "gene": "UniProtKB:Q9UQR1",
  "term_label": "Unknown cellular component"
}